negative regulation of hair follicle cell proliferation [GO:0071337] (biological process) Definition: Any process that stops, prevents or reduces the rate or extent of hair follicle cell proliferation. Sources: GOC:mah Also known as: down regulation of hair follicle cell proliferation, down-regulation of hair follicle cell proliferation, downregulation of hair follicle cell proliferation, inhibition of hair follicle cell proliferation Relationships: is a type of negative regulation of cell population proliferation [GO:0008285]; is a type of regulation of hair follicle cell proliferation [GO:0071336]; negatively regulates hair follicle cell proliferation [GO:0071335]